{
  "term_id": "GO:0033044",
  "term_label": "regulation of chromosome organization",
  "gene_symbol": "CENPV",
  "gene": "UniProtKB:Q7Z7K6",
  "gene_name": "Centromere protein V"
}